{
  "term_id": "UNKNOWN:0001",
  "gene": "UniProtKB:P01732",
  "gene_name": "T-cell surface glycoprotein CD8 alpha chain",
  "gene_symbol": "CD8A",
  "term_label": "Unknown molecular function"
}